protein kinase binding [GO:0019901] (molecular function) Subtypes: protein kinase C binding [GO:0005080], JUN kinase binding [GO:0008432], GO:0031434, mitogen-activated protein kinase kinase kinase binding [GO:0031435], mitogen-activated protein kinase kinase kinase kinase binding [GO:0033161], GO:0034236, protein kinase B binding [GO:0043422], 3-phosphoinositide-dependent protein kinase binding [GO:0043423], protein histidine kinase binding [GO:0043424], mitogen-activated protein kinase binding [GO:0051019], protein serine/threonine kinase binding [GO:0120283], protein tyrosine kinase binding [GO:1990782] Sources: GOC:jl Relationships: is a type of kinase binding [GO:0019900] Definition: Binding to a protein kinase, any enzyme that catalyzes the transfer of a phosphate group, usually from ATP, to a protein substrate.